{
  "term_label": "RNA polymerase II cis-regulatory region sequence-specific DNA binding",
  "gene_symbol": "ZBTB34",
  "gene": "UniProtKB:Q8NCN2",
  "term_id": "GO:0000978",
  "gene_name": "Zinc finger and BTB domain-containing protein 34"
}